{
  "gene_symbol": "ZNF815P",
  "gene": "UniProtKB:A8K554",
  "term_id": "UNKNOWN:0002",
  "term_label": "Unknown biological process",
  "gene_name": "Putative protein ZNF815"
}